culmorin biosynthetic process [GO:0106210] (biological process) References: PMID:19880637, PMID:26673640 Sources: GOC:ach Also known as: culmorin anabolism, culmorin biosynthesis, culmorin formation, culmorin synthesis Definition: The chemical reactions and pathways resulting in the formation of culmorin, a sesquiterpenoid fungal metabolite and mycotoxin produced by some ascomycete species such as Fusarium culmorum, F. graminearum, F. venenatum and Leptosphaeria oraemaris. Relationships: is a type of sesquiterpenoid biosynthetic process [GO:0016106]; is a type of GO:0034312; is a type of mycotoxin biosynthetic process [GO:0043386]; is a type of sesquiterpene biosynthetic process [GO:0051762]; is a type of secondary alcohol biosynthetic process [GO:1902653]